penicillin catabolic process [GO:0042317] (biological process) Also known as: penicillin breakdown, penicillin catabolism, penicillin degradation Sources: GOC:jl, ISBN:0198506732 Definition: The chemical reactions and pathways resulting in the breakdown of any antibiotic that contains the condensed beta-lactamthiazolidine ring system. Subtypes: benzylpenicillin catabolic process [GO:1901087] Relationships: is a type of GO:0030655; is a type of penicillin metabolic process [GO:0042316]; is a type of sulfur compound catabolic process [GO:0044273]; is a type of monocarboxylic acid catabolic process [GO:0072329]; is_a secondary metabolite catabolic process [GO:0090487] Regulation: RO_0002211 by regulation of penicillin catabolic process [GO:0033247]; negatively regulated by GO:0033248; positively regulated by GO:0033249